oxidoreductase activity, acting on the aldehyde or oxo group of donors, disulfide as acceptor [GO:0016624] (molecular function) Definition: Catalysis of an oxidation-reduction (redox) reaction in which an aldehyde or ketone (oxo) group acts as a hydrogen or electron donor and reduces a disulfide. Sources: GOC:jl Also known as: oxidoreductase activity, acting on the aldehyde or oxo group of donors, disulphide as acceptor Relationships: is a type of oxidoreductase activity, acting on the aldehyde or oxo group of donors [GO:0016903] Subtypes: branched-chain 2-oxo acid dehydrogenase activity [GO:0003863], oxoglutarate dehydrogenase (succinyl-transferring) activity [GO:0004591], pyruvate dehydrogenase (acetyl-transferring) activity [GO:0004739], 2-oxoadipate dehydrogenase activity [GO:0160166]